{
  "gene": "UniProtKB:P40261",
  "term_id": "GO:0005829",
  "gene_symbol": "NNMT",
  "term_label": "cytosol",
  "gene_name": "Nicotinamide N-methyltransferase"
}